negative regulation of type I interferon production [GO:0032480] (BP) Sources: GOC:add, GOC:mah Relationships: is a type of negative regulation of cytokine production [GO:0001818]; is_a regulation of type I interferon production [GO:0032479]; negatively regulates type I interferon production [GO:0032606] Subtypes: GO:0032687, negative regulation of interferon-beta production [GO:0032688] Also known as: down regulation of type I interferon production, down-regulation of type I interferon production, downregulation of type I interferon production, negative regulation of type I IFN production, inhibition of type I interferon production Definition: Any process that stops, prevents, or reduces the frequency, rate, or extent of type I interferon production. Type I interferons include the interferon-alpha, beta, delta, episilon, zeta, kappa, tau, and omega gene families.